{
  "gene": "UniProtKB:P20674",
  "gene_symbol": "COX5A",
  "term_label": "mitochondrial electron transport, cytochrome c to oxygen",
  "term_id": "GO:0006123",
  "gene_name": "Cytochrome c oxidase subunit 5A, mitochondrial"
}